indolin-2-one monooxygenase activity [GO:0036191] (molecular function) Definition: Catalysis of the reaction: ndolin-2-one + reduced [NADPH-hemoprotein reductase] + O2 = 3-hydroxyindolin-2-one + oxidized [NADPH-hemoprotein reductase] + H2O + H+. Sources: RHEA:31919 Also known as: indolin-2-one,NAD(P)H:oxygen oxidoreductase (3-hydroxylating) Relationships: is a type of oxidoreductase activity, acting on paired donors, with incorporation or reduction of molecular oxygen, reduced flavin or flavoprotein as one donor, and incorporation of one atom of oxygen [GO:0016712]